{
  "gene": "UniProtKB:P21918",
  "term_label": "G protein-coupled dopamine receptor signaling pathway",
  "gene_symbol": "DRD5",
  "term_id": "GO:0007212",
  "gene_name": "D(1B) dopamine receptor"
}